{
  "gene_symbol": "FAM219B",
  "gene": "UniProtKB:Q5XKK7",
  "term_label": "Unknown molecular function",
  "gene_name": "Protein FAM219B",
  "term_id": "UNKNOWN:0001"
}